{
  "term_id": "GO:0005743",
  "gene_symbol": "MPC2",
  "term_label": "mitochondrial inner membrane",
  "gene_name": "Mitochondrial pyruvate carrier 2",
  "gene": "UniProtKB:O95563"
}